{
  "gene_symbol": "CDIP1",
  "gene_name": "Cell death-inducing p53-target protein 1",
  "term_label": "intrinsic apoptotic signaling pathway in response to DNA damage by p53 class mediator",
  "term_id": "GO:0042771",
  "gene": "UniProtKB:Q9H305"
}